{
  "gene_name": "Zinc finger protein 559",
  "gene_symbol": "ZNF559",
  "gene": "UniProtKB:Q9BR84",
  "term_id": "GO:0000977",
  "term_label": "RNA polymerase II transcription regulatory region sequence-specific DNA binding"
}